lipoprotein transport [GO:0042953] (biological process) Sources: GOC:jl, ISBN:0198506732 Relationships: is a type of protein transport [GO:0015031]; is_a GO:0044872 Regulation: regulated by regulation of lipoprotein transport [GO:0140075]; negatively regulated by negative regulation of lipoprotein transport [GO:0140076]; positively regulated by GO:0140077 Definition: The directed movement of any conjugated, water-soluble protein in which the nonprotein group consists of a lipid or lipids, into, out of or within a cell, or between cells, by means of some agent such as a transporter or pore.